{
  "term_label": "epithelial cell differentiation",
  "gene": "UniProtKB:P08727",
  "gene_symbol": "KRT19",
  "term_id": "GO:0030855",
  "gene_name": "Keratin, type I cytoskeletal 19"
}